{
  "gene": "UniProtKB:P20936",
  "term_id": "GO:0005096",
  "gene_name": "Ras GTPase-activating protein 1",
  "term_label": "GTPase activator activity",
  "gene_symbol": "RASA1"
}